{
  "term_label": "Unknown biological process",
  "gene_name": "Translocon-associated protein subunit gamma",
  "gene_symbol": "SSR3",
  "gene": "UniProtKB:Q9UNL2",
  "term_id": "UNKNOWN:0002"
}